{
  "gene_symbol": "NHLRC1",
  "term_id": "GO:0000209",
  "gene_name": "E3 ubiquitin-protein ligase NHLRC1",
  "term_label": "protein polyubiquitination",
  "gene": "UniProtKB:Q6VVB1"
}